{
  "gene_symbol": "LINS1",
  "gene": "UniProtKB:Q8NG48",
  "term_id": "UNKNOWN:0001",
  "gene_name": "Protein Lines homolog 1",
  "term_label": "Unknown molecular function"
}